{
  "gene_name": "Leucine-rich repeat-containing protein 26",
  "gene_symbol": "LRRC26",
  "term_id": "GO:0099104",
  "term_label": "potassium channel activator activity",
  "gene": "UniProtKB:Q2I0M4"
}